{
  "term_id": "UNKNOWN:0003",
  "gene_name": "Ankyrin repeat domain-containing protein 45",
  "term_label": "Unknown cellular component",
  "gene": "UniProtKB:Q5TZF3",
  "gene_symbol": "ANKRD45"
}